endosomal vesicle fusion [GO:0034058] (biological process) Also known as: endosome vesicle fusion Regulation: negatively regulated by negative regulation of endosomal vesicle fusion [GO:1905362]; positively regulated by positive regulation of endosomal vesicle fusion [GO:1905363]; regulated by GO:1905364 References: PMID:11964142, PMID:9422733 Relationships: is a type of vesicle fusion [GO:0006906] Definition: The homotypic fusion of endocytic vesicles to form or add to an early endosome.